insulin-like growth factor binding protein complex [GO:0016942] (cellular component) Definition: A complex of proteins which includes the insulin-like growth factor (IGF) and a number of IGF-binding proteins. The complex plays a role in growth and development. Subtypes: insulin-like growth factor ternary complex [GO:0042567], GO:0042568 Also known as: IGF binding protein complex Relationships: is a type of growth factor complex [GO:0036454]; is part of extracellular space [GO:0005615] Sources: GOC:jl